{
  "gene_name": "T cell receptor alpha joining 17 (Fragment)",
  "term_label": "Unknown biological process",
  "gene_symbol": "TRAJ17",
  "term_id": "UNKNOWN:0002",
  "gene": "UniProtKB:A0A075B6W8"
}